{
  "term_label": "Unknown biological process",
  "gene_name": "E3 ubiquitin_ISG15 ligase TRIM25",
  "term_id": "UNKNOWN:0002",
  "gene": "UniProtKB:Q14258",
  "gene_symbol": "TRIM25"
}